{
  "gene_symbol": "FHAD1",
  "gene": "UniProtKB:B1AJZ9",
  "term_label": "Unknown cellular component",
  "gene_name": "Forkhead-associated domain-containing protein 1",
  "term_id": "UNKNOWN:0003"
}